{
  "gene_symbol": "CDH2",
  "gene": "UniProtKB:P19022",
  "term_label": "adherens junction",
  "gene_name": "Cadherin-2",
  "term_id": "GO:0005912"
}